{
  "term_label": "nucleus",
  "gene": "UniProtKB:Q9ULX9",
  "gene_symbol": "MAFF",
  "term_id": "GO:0005634",
  "gene_name": "Transcription factor MafF"
}